adrenergic receptor signaling pathway [GO:0071875] (biological process) Relationships: is a type of G protein-coupled receptor signaling pathway [GO:0007186]; has part adrenergic receptor activity [GO:0004935] Definition: A G protein-coupled receptor signaling pathway initiated by a ligand binding to an adrenergic receptor on the surface of a target cell, and ending with the regulation of a downstream cellular process. Also known as: adrenergic receptor signalling pathway, adrenoceptor signaling pathway Subtypes: GO:0071880, adenylate cyclase-inhibiting adrenergic receptor signaling pathway [GO:0071881], phospholipase C-activating adrenergic receptor signaling pathway [GO:0071882], MAPK-activating adrenergic receptor signaling pathway [GO:0071883] Sources: GOC:BHF Regulation: positively regulated by positive regulation of adenylate cyclase-activating adrenergic receptor signaling pathway [GO:0071879]